heme biosynthetic process [GO:0006783] (biological process) Subtypes: heme A biosynthetic process [GO:0006784], heme B biosynthetic process [GO:0006785], heme C biosynthetic process [GO:0006786], siroheme biosynthetic process [GO:0019354], GO:0048034 References: PMID:11788607 Sources: GOC:jl Also known as: haem biosynthesis, haem biosynthetic process, heme anabolism, heme biosynthesis, heme formation, heme synthesis Relationships: is a type of GO:0006779; is a type of heme metabolic process [GO:0042168]; is_a pigment biosynthetic process [GO:0046148] Definition: The chemical reactions and pathways resulting in the formation of heme, any compound of iron complexed in a porphyrin (tetrapyrrole) ring, from less complex precursors. Regulation: regulated by GO:0070453; negatively regulated by GO:0070454; positively regulated by positive regulation of heme biosynthetic process [GO:0070455]